myofibroblast cell apoptotic process [GO:1904516] (biological process) Also known as: MFB apoptotic process, MFB apoptosis, myofibroblast cell apoptosis Definition: Any apoptotic process in a myofibroblast cell. Relationships: is a type of apoptotic process [GO:0006915] Regulation: regulated by regulation of myofibroblast cell apoptotic process [GO:1904520]; negatively regulated by negative regulation of myofibroblast cell apoptotic process [GO:1904521]; positively regulated by positive regulation of myofibroblast cell apoptotic process [GO:1904522] References: PMID:23026405 Sources: GOC:TermGenie, GO_REF:0000085